{
  "term_label": "cytosol",
  "gene_name": "Elongator complex protein 1",
  "gene_symbol": "ELP1",
  "term_id": "GO:0005829",
  "gene": "UniProtKB:O95163"
}